{
  "gene": "UniProtKB:Q86YW5",
  "term_id": "GO:0005886",
  "term_label": "plasma membrane",
  "gene_name": "Trem-like transcript 1 protein",
  "gene_symbol": "TREML1"
}